{
  "gene_symbol": "SERPING1",
  "gene_name": "Plasma protease C1 inhibitor",
  "term_label": "Unknown biological process",
  "term_id": "UNKNOWN:0002",
  "gene": "UniProtKB:P05155"
}